{
  "gene": "UniProtKB:Q9NS87",
  "gene_symbol": "KIF15",
  "term_label": "ATP hydrolysis activity",
  "term_id": "GO:0016887",
  "gene_name": "Kinesin-like protein KIF15"
}